{
  "gene_name": "Rhomboid domain-containing protein 3",
  "gene_symbol": "RHBDD3",
  "term_id": "UNKNOWN:0002",
  "gene": "UniProtKB:Q9Y3P4",
  "term_label": "Unknown biological process"
}